{
  "gene_symbol": "SERPINB6",
  "gene_name": "Serpin B6",
  "term_label": "Unknown biological process",
  "term_id": "UNKNOWN:0002",
  "gene": "UniProtKB:P35237"
}